{
  "gene_name": "Glutamate receptor ionotropic, delta-1",
  "gene_symbol": "GRID1",
  "term_id": "GO:0043197",
  "term_label": "dendritic spine",
  "gene": "UniProtKB:Q9ULK0"
}